polysaccharide binding [GO:0030247] (molecular function) Sources: GOC:mah Relationships: is a type of carbohydrate binding [GO:0030246] Definition: Binding to a polysaccharide, a polymer of many (typically more than 10) monosaccharide residues linked glycosidically. Also known as: polysaccharide assembly with MHC class II protein complex Subtypes: (1->3)-beta-D-glucan binding [GO:0001872], heteropolysaccharide binding [GO:0010297], GO:0030248, cellodextrin binding [GO:0044584], GO:0048028, xylan binding [GO:2001062], mannan binding [GO:2001065], GO:2001067, glycogen binding [GO:2001069], starch binding [GO:2001070], cyclodextrin binding [GO:2001073], (1->3),(1->4)-beta-glucan binding [GO:2001077], GO:2001078, (1->4)-beta-D-galactan binding [GO:2001081], inulin binding [GO:2001082], GO:2001083, arabinogalactan binding [GO:2001085]